{
  "term_label": "protein kinase binding",
  "gene_symbol": "RAC2",
  "term_id": "GO:0019901",
  "gene": "UniProtKB:P15153",
  "gene_name": "Ras-related C3 botulinum toxin substrate 2"
}